{
  "term_label": "Golgi membrane",
  "gene_symbol": "MAN1A1",
  "term_id": "GO:0000139",
  "gene": "UniProtKB:P33908",
  "gene_name": "Mannosyl-oligosaccharide 1,2-alpha-mannosidase IA"
}